{
  "gene": "UniProtKB:Q16778",
  "gene_symbol": "H2BC21",
  "gene_name": "Histone H2B type 2-E",
  "term_label": "structural constituent of chromatin",
  "term_id": "GO:0030527"
}